{
  "term_label": "nucleus",
  "gene_symbol": "AFG2B",
  "term_id": "GO:0005634",
  "gene": "UniProtKB:Q9BVQ7",
  "gene_name": "ATPase family gene 2 protein homolog B"
}